{
  "term_label": "intermediate filament organization",
  "gene": "UniProtKB:P13647",
  "term_id": "GO:0045109",
  "gene_symbol": "KRT5",
  "gene_name": "Keratin, type II cytoskeletal 5"
}